{
  "gene_name": "Protein SIX6OS1",
  "gene": "UniProtKB:Q8N1H7",
  "term_id": "UNKNOWN:0001",
  "gene_symbol": "SIX6OS1",
  "term_label": "Unknown molecular function"
}